{
  "gene_symbol": "KNDC1",
  "term_label": "dendrite",
  "gene_name": "Kinase non-catalytic C-lobe domain-containing protein 1",
  "term_id": "GO:0030425",
  "gene": "UniProtKB:Q76NI1"
}